{
  "gene_symbol": "RHBDF1",
  "term_label": "Unknown molecular function",
  "gene": "UniProtKB:Q96CC6",
  "term_id": "UNKNOWN:0001",
  "gene_name": "Inactive rhomboid protein 1"
}